{
  "gene": "UniProtKB:Q96PG8",
  "gene_name": "Bcl-2-binding component 3, isoforms 3_4",
  "term_id": "UNKNOWN:0001",
  "term_label": "Unknown molecular function",
  "gene_symbol": "BBC3"
}